cell-cell signaling involved in placenta development [GO:0060673] (biological process) Also known as: cell-cell signalling involved in placenta development Definition: Any process that mediates the transfer of information from one cell to another. References: PMID:16916377 Sources: GOC:dph Relationships: is a type of cell-cell signaling [GO:0007267]; is part of embryonic placenta development [GO:0001892]